multi-pass translocon complex [GO:0160064] (cellular component) Relationships: is a type of ER membrane insertion complex [GO:0072379] Also known as: MPT complex, TMCO1 translocon References: PMID:36261522, PMID:36261528 Definition: A protein complex that mediates the insertion of multi-pass transmembrane proteins into endoplasmic reticulum (ER) membrane. Substrates enter via the lateral gate of the Sec61 translocon. The complex comprises the GEL subcomplex (composed of RAB5IF/OPTI and TMCO1), the BOS subcomplex (composed of NCLN/Nicalin, NOMO and TMEM147) and the PAT subcomplex (composed of WDR83OS/Asterix and CCDC47).